regulation of fumonisin biosynthetic process [GO:1900683] (biological process) Sources: GOC:TermGenie, GOC:di Subtypes: negative regulation of fumonisin biosynthetic process [GO:1900684], GO:1900685 Also known as: regulation of fumonisin anabolism, regulation of fumonisin biosynthesis, regulation of fumonisin formation, regulation of fumonisin synthesis Relationships: is a type of regulation of ketone metabolic process [GO:0010565]; is a type of regulation of small molecule metabolic process [GO:0062012]; is_a regulation of secondary metabolite biosynthetic process [GO:1900376]; regulates GO:1900541 Definition: Any process that modulates the frequency, rate or extent of fumonisin biosynthetic process.